cellular response to salt [GO:1902075] (biological process) Subtypes: GO:1903936, cellular response to sodium phosphate [GO:1904384] Also known as: cellular response to salinity Relationships: is a type of cellular response to chemical stimulus [GO:0070887]; is a type of response to salt [GO:1902074] References: PMID:16666921 Sources: GOC:TermGenie, GOC:mls Definition: Any process that results in a change in state or activity of a cell (in terms of movement, secretion, enzyme production, gene expression, etc.) as a result of a salt stimulus.